{
  "gene_name": "Protocadherin gamma-A7",
  "term_id": "GO:0007155",
  "term_label": "cell adhesion",
  "gene_symbol": "PCDHGA7",
  "gene": "UniProtKB:Q9Y5G6"
}